{
  "gene_name": "tRNA methyltransferase 10 homolog A",
  "term_label": "nucleoplasm",
  "gene_symbol": "TRMT10A",
  "term_id": "GO:0005654",
  "gene": "UniProtKB:Q8TBZ6"
}